{
  "gene": "UniProtKB:P23229",
  "gene_name": "Integrin alpha-6",
  "term_label": "cell-cell adhesion",
  "gene_symbol": "ITGA6",
  "term_id": "GO:0098609"
}